{
  "gene_symbol": "EN2",
  "term_id": "GO:0000978",
  "gene": "UniProtKB:P19622",
  "gene_name": "Homeobox protein engrailed-2",
  "term_label": "RNA polymerase II cis-regulatory region sequence-specific DNA binding"
}